{
  "gene": "UniProtKB:P04083",
  "gene_name": "Annexin A1",
  "term_id": "GO:0005634",
  "gene_symbol": "ANXA1",
  "term_label": "nucleus"
}